{
  "term_id": "GO:0001518",
  "gene_name": "Sodium channel protein type 5 subunit alpha",
  "term_label": "voltage-gated sodium channel complex",
  "gene_symbol": "SCN5A",
  "gene": "UniProtKB:Q14524"
}